{
  "term_id": "GO:0005847",
  "gene_name": "RNA polymerase II subunit A C-terminal domain phosphatase SSU72 like protein 6",
  "gene_symbol": "SSU72L6",
  "gene": "UniProtKB:A0A1W2PR75",
  "term_label": "mRNA cleavage and polyadenylation specificity factor complex"
}